CD8-positive, alpha-beta cytotoxic T cell differentiation [GO:0002308] (BP) Definition: The process in which a precursor cell type acquires the specialized features of a CD8-positive, alpha-beta cytotoxic T cell. Also known as: CD8-positive, alpha-beta cytotoxic T lymphocyte differentiation, CD8-positive, alpha-beta cytotoxic T-cell differentiation, CD8-positive, alpha-beta cytotoxic T-lymphocyte differentiation, CD8-positive, alpha-beta cytotoxic T cell development Relationships: is a type of CD8-positive, alpha-beta T cell differentiation [GO:0043374]; is a type of cytotoxic T cell differentiation [GO:0045065] Sources: GOC:add, ISBN:0781735149 Note: Note that immunologists typically use the word 'development' to refer to cells of B or T cell lineages undergoing the process that GO describes as 'cell differentiation'.